{
  "term_label": "RNA polymerase II cis-regulatory region sequence-specific DNA binding",
  "gene_symbol": "MIXL1",
  "term_id": "GO:0000978",
  "gene_name": "Homeobox protein MIXL1",
  "gene": "UniProtKB:Q9H2W2"
}